purine-containing compound salvage [GO:0043101] (biological process) Relationships: is a type of GO:0043094; is a type of purine-containing compound biosynthetic process [GO:0072522] Definition: Any process that generates a purine-containing compound, any nucleobase, nucleoside, nucleotide or nucleic acid that contains a purine base, from derivatives of them without de novo synthesis. Also known as: purine salvage Sources: GOC:jl Subtypes: purine ribonucleoside salvage [GO:0006166], purine nucleotide salvage [GO:0032261], GO:0043096, purine deoxyribonucleoside salvage [GO:0043098]